{
  "gene_name": "BTB_POZ domain-containing protein KCTD21",
  "gene": "UniProtKB:Q4G0X4",
  "term_label": "ubiquitin-dependent protein catabolic process",
  "term_id": "GO:0006511",
  "gene_symbol": "KCTD21"
}